{
  "term_id": "GO:0019005",
  "gene": "UniProtKB:Q8IY45",
  "gene_name": "Protein AMN1 homolog",
  "gene_symbol": "AMN1",
  "term_label": "SCF ubiquitin ligase complex"
}